{
  "term_id": "GO:0005125",
  "gene": "UniProtKB:O43557",
  "gene_symbol": "TNFSF14",
  "term_label": "cytokine activity",
  "gene_name": "Tumor necrosis factor ligand superfamily member 14"
}